positive regulation of actin filament annealing [GO:0110056] (biological process) References: PMID:10585915, PMID:11575927, PMID:19244341 Sources: GOC:mah Definition: Any process that activates or increases the frequency, rate or extent of actin filament annealing, i.e. the end-to-end joining of existing actin filaments. Relationships: is a type of regulation of actin filament annealing [GO:0110054]